inflorescence meristem growth [GO:0010450] (biological process) Sources: GOC:tb Regulation: regulated by GO:0010081 Definition: The increase in size or mass of an inflorescence meristem, a population of undifferentiated cells in a plant shoot which produces small leaves and then floral meristems, which will give rise to flowers. Relationships: is_a developmental process involved in reproduction [GO:0003006]; is a type of meristem growth [GO:0035266]; is part of GO:0010229